{
  "gene": "UniProtKB:Q96EU6",
  "gene_symbol": "RRP36",
  "term_id": "UNKNOWN:0001",
  "term_label": "Unknown molecular function",
  "gene_name": "Ribosomal RNA processing protein 36 homolog"
}